histone H3K18 acetyltransferase activity [GO:0043993] (molecular function) References: PMID:18552846 Note: Comment: Note that the residue position corresponds to the canonical human H3 histone (UniProtKB:P84243); this residue is conserved across all eukaryotes. Residue 1 is the first residue following removal of the initiating Methionine (Met). Note that each histone is encoded by multiple genes, and sequences may vary across different genes within an organism. Also known as: histone H3-K18 acetyltransferase activity, histone acetylase activity (H3-K18 specific), histone acetyltransferase activity (H3-K18 specific), histone lysine N-acetyltransferase activity (H3-K18 specific) Relationships: is_a GO:0010484 Definition: Catalysis of the reaction: acetyl-CoA + histone H3 L-lysine (position 18) = CoA + histone H3 N6-acetyl-L-lysine (position 18).